{
  "gene": "UniProtKB:Q9BZF1",
  "term_label": "cytosol",
  "term_id": "GO:0005829",
  "gene_symbol": "OSBPL8",
  "gene_name": "Oxysterol-binding protein-related protein 8"
}